{
  "gene": "UniProtKB:Q9H069",
  "gene_symbol": "DRC3",
  "gene_name": "Dynein regulatory complex subunit 3",
  "term_label": "Unknown biological process",
  "term_id": "UNKNOWN:0002"
}